extrinsic component of Golgi membrane [GO:0090498] (cellular component) Definition: The component of a Golgi membrane consisting of gene products and protein complexes that are loosely bound to one of its surfaces, but not integrated into the hydrophobic region. References: PMID:21337012 Sources: GOC:dos Also known as: extrinsic to Golgi membrane Relationships: is a type of extrinsic component of organelle membrane [GO:0031312]; is part of Golgi membrane [GO:0000139]